{
  "gene_name": "Peptidyl-prolyl cis-trans isomerase A",
  "term_label": "protein folding",
  "gene_symbol": "PPIA",
  "term_id": "GO:0006457",
  "gene": "UniProtKB:P62937"
}